{
  "gene_symbol": "TOP3B",
  "gene_name": "DNA topoisomerase 3-beta-1",
  "term_label": "nucleus",
  "term_id": "GO:0005634",
  "gene": "UniProtKB:O95985"
}